{
  "term_label": "Unknown molecular function",
  "term_id": "UNKNOWN:0001",
  "gene": "UniProtKB:Q9NZV5",
  "gene_name": "Selenoprotein N",
  "gene_symbol": "SELENON"
}